{
  "gene": "UniProtKB:Q8IVF2",
  "term_id": "GO:0043484",
  "gene_name": "Protein AHNAK2",
  "gene_symbol": "AHNAK2",
  "term_label": "regulation of RNA splicing"
}